{
  "gene": "UniProtKB:Q13621",
  "term_label": "apical plasma membrane",
  "gene_symbol": "SLC12A1",
  "gene_name": "Solute carrier family 12 member 1",
  "term_id": "GO:0016324"
}